{
  "gene_name": "Transmembrane protein 140",
  "term_id": "UNKNOWN:0002",
  "term_label": "Unknown biological process",
  "gene": "UniProtKB:Q9NV12",
  "gene_symbol": "TMEM140"
}